peroxisome matrix targeting signal-1 binding [GO:0005052] (molecular function) Definition: Binding to a type 1 peroxisome targeting signal, a tripeptide with the consensus sequence (S/A/C)-(K/R/H)-L. Also known as: PTS1 binding, peroxisomal targeting signal 1 (PTS1) binding, peroxisome targeting signal-1 binding, PEX5, PTS1 receptor, peroxisome targeting signal-1 receptor References: PMID:11687502 Sources: GOC:mah Relationships: is a type of GO:0000268